{
  "gene": "UniProtKB:Q9H1C7",
  "gene_name": "Cysteine-rich and transmembrane domain-containing protein 1",
  "gene_symbol": "CYSTM1",
  "term_id": "UNKNOWN:0002",
  "term_label": "Unknown biological process"
}